{
  "term_id": "GO:0003684",
  "gene_symbol": "NBN",
  "gene_name": "Nibrin",
  "term_label": "damaged DNA binding",
  "gene": "UniProtKB:O60934"
}